venous endothelial cell differentiation [GO:0060843] (biological process) Definition: The process in which a relatively unspecialized endothelial cell acquires specialized features of a venous endothelial cell, a thin flattened cell that lines the inside surfaces of veins. Relationships: is_a GO:0060837 Sources: GOC:dph, GOC:sdb_2009, GOC:tb